{
  "gene_symbol": "SLC17A4",
  "gene_name": "Probable small intestine urate exporter",
  "term_label": "transmembrane transporter activity",
  "term_id": "GO:0022857",
  "gene": "UniProtKB:Q9Y2C5"
}